{
  "gene_name": "Clusterin-associated protein 1",
  "gene_symbol": "CLUAP1",
  "term_id": "GO:0005929",
  "gene": "UniProtKB:Q96AJ1",
  "term_label": "cilium"
}